{
  "gene": "UniProtKB:Q6NUJ1",
  "term_id": "GO:0019216",
  "term_label": "regulation of lipid metabolic process",
  "gene_name": "Proactivator polypeptide-like 1",
  "gene_symbol": "PSAPL1"
}